{
  "term_id": "GO:0000978",
  "gene_name": "Nucleus accumbens-associated protein 1",
  "term_label": "RNA polymerase II cis-regulatory region sequence-specific DNA binding",
  "gene_symbol": "NACC1",
  "gene": "UniProtKB:Q96RE7"
}